regulation of myoblast proliferation [GO:2000291] (biological process) Definition: Any process that modulates the frequency, rate or extent of myoblast proliferation. Sources: GOC:mah Relationships: is a type of regulation of cell population proliferation [GO:0042127]; regulates myoblast proliferation [GO:0051450] Subtypes: regulation of cardiac muscle myoblast proliferation [GO:0110022], positive regulation of myoblast proliferation [GO:2000288], GO:2000818